{
  "gene": "UniProtKB:A0A087WXS9",
  "gene_symbol": "TBC1D3I",
  "term_label": "GTPase activator activity",
  "gene_name": "TBC1 domain family member 3I",
  "term_id": "GO:0005096"
}